{
  "term_id": "GO:0004222",
  "gene": "UniProtKB:Q9BXP8",
  "term_label": "metalloendopeptidase activity",
  "gene_symbol": "PAPPA2",
  "gene_name": "Pappalysin-2"
}